{
  "gene_symbol": "SLMAP",
  "gene_name": "Sarcolemmal membrane-associated protein",
  "term_label": "negative regulation of hippo signaling",
  "gene": "UniProtKB:Q14BN4",
  "term_id": "GO:0035331"
}